{
  "term_id": "GO:0008420",
  "gene_name": "RNA polymerase II subunit A C-terminal domain phosphatase SSU72 like protein 6",
  "gene_symbol": "SSU72L6",
  "term_label": "RNA polymerase II CTD heptapeptide repeat phosphatase activity",
  "gene": "UniProtKB:A0A1W2PR75"
}